branching morphogenesis of an epithelial tube [GO:0048754] (biological process) Relationships: is a type of tube morphogenesis [GO:0035239]; is a type of morphogenesis of a branching epithelium [GO:0061138]; is part of epithelial tube morphogenesis [GO:0060562] Definition: The process in which the anatomical structures of branches in an epithelial tube are generated and organized. A tube is a long hollow cylinder. Also known as: tubulogenesis Subtypes: branching involved in blood vessel morphogenesis [GO:0001569], branching involved in ureteric bud morphogenesis [GO:0001658], epithelial tube branching involved in lung morphogenesis [GO:0060441], GO:0060444, branching involved in open tracheal system development [GO:0060446], branching involved in lymph vessel morphogenesis [GO:0060854] Sources: GOC:dgh, GOC:dph, GOC:jid